{
  "term_id": "GO:0032233",
  "gene": "UniProtKB:Q9H987",
  "gene_symbol": "SYNPO2L",
  "term_label": "positive regulation of actin filament bundle assembly",
  "gene_name": "Synaptopodin 2-like protein"
}